{
  "gene_symbol": "TRIM28",
  "term_label": "ubiquitin protein ligase activity",
  "gene": "UniProtKB:Q13263",
  "term_id": "GO:0061630",
  "gene_name": "Transcription intermediary factor 1-beta"
}